membraneless organelle [GO:0043228] (cellular component) Relationships: is a type of GO:0043226 Sources: GOC:go_curators Definition: Organized structure of distinctive morphology and function, not bounded by a lipid bilayer membrane. Includes ribosomes, the cytoskeleton and chromosomes. Also known as: membrane-less organelle, non-membrane-bounded organelle, non-membrane-enclosed organelle, biological condensate Subtypes: bacterial-type flagellum [GO:0009288], intracellular membraneless organelle [GO:0043232], GO:0043264, archaeal-type flagellum [GO:0097589]